CX3C chemokine receptor binding [GO:0031737] (molecular function) Definition: Binding to a CX3C chemokine receptor. Sources: GOC:mah, GOC:nln Relationships: is a type of chemokine receptor binding [GO:0042379] Also known as: fractalkine receptor binding, CX3C chemokine receptor ligand